{
  "gene_symbol": "CTSO",
  "gene_name": "Cathepsin O",
  "term_label": "extracellular space",
  "term_id": "GO:0005615",
  "gene": "UniProtKB:P43234"
}